zinc ion transport [GO:0006829] (biological process) Subtypes: GO:0071577 Regulation: regulated by GO:0071579; negatively regulated by negative regulation of zinc ion transport [GO:0071582] Relationships: is a type of transition metal ion transport [GO:0000041] Also known as: zinc II ion transport, zinc transport Sources: GOC:ai Definition: The directed movement of zinc (Zn II) ions into, out of or within a cell, or between cells, by means of some agent such as a transporter or pore.